(-)-menthol monooxygenase activity [GO:0047505] (MF) Sources: EC:1.14.13.46, RHEA:11648 Also known as: (-)-menthol,NADPH:oxygen oxidoreductase (8-hydroxylating), l-menthol monooxygenase activity Relationships: is a type of oxidoreductase activity, acting on paired donors, with incorporation or reduction of molecular oxygen, NAD(P)H as one donor, and incorporation of one atom of oxygen [GO:0016709] Definition: Catalysis of the reaction: (-)-menthol + H+ + NADPH + O2 = 1,4-menthane-3,8-diol + H2O + NADP+.